cranial ganglion development [GO:0061550] (biological process) Also known as: cranial ganglia development Sources: GOC:dph Subtypes: lateral line ganglion development [GO:0048890], trigeminal ganglion development [GO:0061551], facioacoustic ganglion development [GO:1903375] Relationships: is a type of ganglion development [GO:0061548]; is part of cranial nerve development [GO:0021545] Definition: The process whose specific outcome is the progression of a cranial ganglion over time, from its formation to the mature structure.